{
  "gene_symbol": "ZNF652",
  "term_id": "GO:0000981",
  "gene_name": "Zinc finger protein 652",
  "gene": "UniProtKB:Q9Y2D9",
  "term_label": "DNA-binding transcription factor activity, RNA polymerase II-specific"
}